{
  "term_id": "GO:0042742",
  "term_label": "defense response to bacterium",
  "gene_name": "Extracellular glycoprotein lacritin",
  "gene": "UniProtKB:Q9GZZ8",
  "gene_symbol": "LACRT"
}